{
  "term_label": "negative regulation of actin nucleation",
  "gene": "UniProtKB:Q7Z6K5",
  "gene_name": "Arpin",
  "term_id": "GO:0051126",
  "gene_symbol": "ARPIN"
}